{
  "gene_name": "Ribitol 5-phosphate transferase FKRP",
  "gene_symbol": "FKRP",
  "term_label": "protein O-linked glycosylation via mannose",
  "gene": "UniProtKB:Q9H9S5",
  "term_id": "GO:0035269"
}